positive regulation of tumor necrosis factor production [GO:0032760] (biological process) Definition: Any process that activates or increases the frequency, rate or extent of tumor necrosis factor production. References: PMID:10891884, PMID:15560120 Sources: GOC:TermGenie, GO_REF:0000058 Also known as: positive regulation of TNF production, positive regulation of TNF-alpha production, positive regulation of tumor necrosis factor-alpha production, up regulation of tumor necrosis factor production, up-regulation of tumor necrosis factor production, upregulation of tumor necrosis factor production, activation of tumor necrosis factor production, positive regulation of TNF secretion, positive regulation of cachectin secretion, positive regulation of tumor necrosis factor biosynthesis, positive regulation of tumor necrosis factor biosynthetic process, positive regulation of tumor necrosis factor formation, positive regulation of tumor necrosis factor secretion, stimulation of tumor necrosis factor production Note: Note that this term refers only to the specific, original 'tumor necrosis factor' protein (TNF) and not other members of the tumor necrosis factor superfamily (those with the gene symbol root 'TNFSF'). Relationships: is a type of regulation of tumor necrosis factor production [GO:0032680]; is a type of GO:1903557; RO_0002213 GO:0032640